{
  "term_label": "extracellular space",
  "gene": "UniProtKB:P41271",
  "term_id": "GO:0005615",
  "gene_symbol": "NBL1",
  "gene_name": "Neuroblastoma suppressor of tumorigenicity 1"
}